{
  "gene": "UniProtKB:P59074",
  "term_id": "GO:0000815",
  "gene_name": "Putative charged multivesicular body protein 4B-like protein CHMP4BP1",
  "term_label": "ESCRT III complex",
  "gene_symbol": "CHMP4BP1"
}